ATF6-mediated unfolded protein response [GO:0036500] (biological process) References: PMID:22013210 Sources: GOC:PARL, GOC:bf Also known as: ATF6 signal transduction pathway, ATF6 branch of UPR, UPR signaling by ATF6 stress sensor, activating transcription factor 6 signaling in unfolded protein response, endoplasmic reticulum unfolded protein response; ATF6 signaling, ATF6-alpha UPR branch, ATF6-beta UPR branch, ATF6 signaling in response to endoplasmic reticulum stress Definition: The series of molecular signals mediated by the endoplasmic reticulum membrane stress sensor ATF6 (activating transcription factor 6). Begins with activation of ATF6 in response to endoplasmic reticulum (ER) stress, and ends with regulation of a downstream cellular process, e.g. transcription. Under conditions of endoplasmic reticulum stress, ATF6 translocates to the Golgi where it is processed by proteases to release a cytoplasmic domain (ATF6f), which operates as a transcriptional activator of many genes required to restore folding capacity. Regulation: regulated by regulation of ATF6-mediated unfolded protein response [GO:1903891]; negatively regulated by negative regulation of ATF6-mediated unfolded protein response [GO:1903892]; positively regulated by GO:1903893 Relationships: is a type of GO:0006984; is_a endoplasmic reticulum unfolded protein response [GO:0030968]